{
  "term_label": "postsynaptic density",
  "gene_symbol": "TMEM108",
  "gene": "UniProtKB:Q6UXF1",
  "term_id": "GO:0014069",
  "gene_name": "Transmembrane protein 108"
}